{
  "term_id": "GO:0005737",
  "gene_symbol": "CASP5",
  "gene_name": "Caspase-5",
  "gene": "UniProtKB:P51878",
  "term_label": "cytoplasm"
}